actin monomer binding [GO:0003785] (molecular function) Definition: Binding to monomeric actin, also known as G-actin. Sources: GOC:ai Also known as: G actin binding Relationships: is a type of actin binding [GO:0003779]